{
  "term_label": "signal transduction",
  "gene_symbol": "BEX2",
  "gene": "UniProtKB:Q9BXY8",
  "term_id": "GO:0007165",
  "gene_name": "Protein BEX2"
}